cellular response to sulfate starvation [GO:0009970] (biological process) Relationships: is a type of cellular response to starvation [GO:0009267] Definition: Any process that results in a change in state or activity of a cell (in terms of movement, secretion, enzyme production, gene expression, etc.) as a result of deprivation of sulfate. Sources: GOC:sm Also known as: cellular response to sulphate starvation